response to endoplasmic reticulum stress [GO:0034976] (biological process) Subtypes: ER overload response [GO:0006983], endoplasmic reticulum unfolded protein response [GO:0030968], ERAD pathway [GO:0036503], endoplasmic reticulum stress-induced pre-emptive quality control [GO:0061857], GO:0070059, response to manganese-induced endoplasmic reticulum stress [GO:1990737] Sources: GOC:cjm, GOC:mah Relationships: is a type of cellular response to stress [GO:0033554] Definition: Any process that results in a change in state or activity of a cell (in terms of movement, secretion, enzyme production, gene expression, etc.) as a result of a stress acting at the endoplasmic reticulum. ER stress usually results from the accumulation of unfolded or misfolded proteins in the ER lumen. Regulation: negatively regulated by negative regulation of response to endoplasmic reticulum stress [GO:1903573]; regulated by regulation of response to endoplasmic reticulum stress [GO:1905897]; positively regulated by positive regulation of response to endoplasmic reticulum stress [GO:1905898] Also known as: ER stress response, cellular response to endoplasmic reticulum stress, response to ER stress